{
  "term_label": "Unknown cellular component",
  "gene": "UniProtKB:Q8NDZ0",
  "term_id": "UNKNOWN:0003",
  "gene_symbol": "BEND2",
  "gene_name": "BEN domain-containing protein 2"
}